{
  "gene": "UniProtKB:P33981",
  "term_id": "GO:0004712",
  "gene_symbol": "TTK",
  "term_label": "protein serine/threonine/tyrosine kinase activity",
  "gene_name": "Dual specificity protein kinase TTK"
}